protein import into nucleus [GO:0006606] (biological process) Definition: The directed movement of a protein from the cytoplasm to the nucleus. Sources: GOC:jl Also known as: establishment of protein localization to nucleus, protein import into cell nucleus, protein nucleus import, protein transport from cytoplasm to nucleus Relationships: is a type of intracellular protein transport [GO:0006886]; is a type of protein localization to nucleus [GO:0034504]; is a type of import into nucleus [GO:0051170]; is a type of establishment of protein localization to organelle [GO:0072594] Subtypes: GO:0006607, ribosomal protein import into nucleus [GO:0006610] Regulation: regulated by GO:0042306; positively regulated by positive regulation of protein import into nucleus [GO:0042307]; negatively regulated by GO:0042308